{
  "gene_name": "Serine protease inhibitor Kazal-type 4",
  "gene": "UniProtKB:O60575",
  "term_id": "UNKNOWN:0001",
  "gene_symbol": "SPINK4",
  "term_label": "Unknown molecular function"
}